{
  "gene_symbol": "FOXH1",
  "gene_name": "Forkhead box protein H1",
  "gene": "UniProtKB:O75593",
  "term_id": "GO:0000976",
  "term_label": "transcription cis-regulatory region binding"
}